{
  "gene_symbol": "NR1H3",
  "gene_name": "Oxysterols receptor LXR-alpha",
  "term_id": "GO:0090575",
  "term_label": "RNA polymerase II transcription regulator complex",
  "gene": "UniProtKB:Q13133"
}